transcription export complex 2 [GO:0070390] (cellular component) References: PMID:17786152, PMID:19289793, PMID:28334829 Sources: GOC:dgf, GOC:mah Relationships: is_a GO:0140513 Also known as: Sac3-Thp1-Sus1-Sem1-Cdc31 complex, TREX-2 complex Definition: A protein complex that couples SAGA-dependent gene expression to mRNA export at the inner side of the nuclear pore complex (NPC). The TREX-2 complex is tethered to the inner side of the NPC via the nucleoporins Nup1 and Nup60; in S. cerevisiae it contains Sac3p, Thp1p, Sem1, Sus1p and Cdc31p.